{
  "term_id": "GO:0030520",
  "gene_symbol": "ESR1",
  "term_label": "estrogen receptor signaling pathway",
  "gene": "UniProtKB:P03372",
  "gene_name": "Estrogen receptor"
}